dihydroorotate dehydrogenase (fumarate) activity [GO:1990663] (molecular function) Definition: Catalysis of the reaction: (S)-dihydroorotate + fumarate = orotate + succinate. References: PMID:1409592 Sources: RHEA:30059 Relationships: is a type of dihydroorotate dehydrogenase activity [GO:0004152]